{
  "gene_name": "Gamma-aminobutyric acid receptor-associated protein-like 1",
  "term_label": "mitophagy",
  "term_id": "GO:0000423",
  "gene": "UniProtKB:Q9H0R8",
  "gene_symbol": "GABARAPL1"
}